type III terminal bouton [GO:0097467] (cellular component) Definition: Terminal inflated portion of the axon of a non-glutamatergic neuron, containing the specialized apparatus necessary to release neurotransmitters at a regulatory synapse. The axon terminus is considered to be the whole region of thickening and the terminal bouton is a specialized region of it. Type III terminal boutons are larger than type II ones. References: PMID:10218156 Sources: GOC:mc Also known as: type III terminal button Relationships: is a type of terminal bouton [GO:0043195]